indole-3-acetaldehyde oxidase activity [GO:0050302] (MF) Sources: RHEA:16277 Also known as: (indol-3-yl)acetaldehyde:oxygen oxidoreductase activity, AO1, IAA oxidase activity, IAAld oxidase activity, indole-3-acetaldehyde:oxygen oxidoreductase activity, indoleacetaldehyde oxidase activity Definition: Catalysis of the reaction: H2O + indole-3-acetaldehyde + O2 = (indol-3-yl)acetate + H+ + H2O2. Relationships: is a type of GO:0018488